{
  "gene_symbol": "STX17",
  "term_id": "GO:0005886",
  "term_label": "plasma membrane",
  "gene": "UniProtKB:P56962",
  "gene_name": "Syntaxin-17"
}